{
  "gene_name": "Signal transducer and activator of transcription 5B",
  "gene": "UniProtKB:P51692",
  "gene_symbol": "STAT5B",
  "term_id": "GO:0000981",
  "term_label": "DNA-binding transcription factor activity, RNA polymerase II-specific"
}